{
  "term_label": "cytoplasm",
  "gene": "UniProtKB:P40123",
  "term_id": "GO:0005737",
  "gene_name": "Adenylyl cyclase-associated protein 2",
  "gene_symbol": "CAP2"
}